{
  "gene_symbol": "GZMH",
  "gene": "UniProtKB:P20718",
  "gene_name": "Granzyme H",
  "term_id": "GO:0005615",
  "term_label": "extracellular space"
}